{
  "gene_name": "Synaptogyrin-4",
  "gene": "UniProtKB:O95473",
  "term_id": "UNKNOWN:0001",
  "term_label": "Unknown molecular function",
  "gene_symbol": "SYNGR4"
}